nitrate reductase (quinone) activity [GO:0160182] (molecular function) Relationships: is a type of nitrate reductase activity [GO:0008940] Sources: RHEA:56144 Also known as: dissimilatory nitrate reductase, dissimilatory nitrate reductase activity, nitrate reductase A activity, nitrate reductase Z activity, quinol-nitrate oxidoreductase activity Definition: Catalysis of the reaction: a quinol + nitrate = a quinone + H2O + nitrite.